{
  "term_label": "basolateral plasma membrane",
  "term_id": "GO:0016323",
  "gene_symbol": "CFTR",
  "gene": "UniProtKB:P13569",
  "gene_name": "Cystic fibrosis transmembrane conductance regulator"
}